{
  "gene": "UniProtKB:Q9NWS8",
  "gene_name": "Required for meiotic nuclear division protein 1 homolog",
  "gene_symbol": "RMND1",
  "term_label": "Unknown molecular function",
  "term_id": "UNKNOWN:0001"
}